{
  "term_label": "cell surface",
  "term_id": "GO:0009986",
  "gene_symbol": "TYROBP",
  "gene": "UniProtKB:O43914",
  "gene_name": "TYRO protein tyrosine kinase-binding protein"
}